{
  "gene": "UniProtKB:Q86XR2",
  "term_id": "UNKNOWN:0002",
  "gene_name": "Protein Niban 3",
  "term_label": "Unknown biological process",
  "gene_symbol": "NIBAN3"
}